aconitate hydratase activity [GO:0003994] (molecular function) Also known as: citrate hydro-lyase activity, aconitase activity, cis-aconitase activity, citrate(isocitrate) hydro-lyase (cis-aconitate-forming), citrate(isocitrate) hydro-lyase activity Sources: EC:4.2.1.3, GOC:pde, GOC:vw Relationships: is a type of hydro-lyase activity [GO:0016836] Definition: Catalysis of the reaction: citrate = isocitrate. The reaction occurs in two steps: (1) citrate = cis-aconitate + H2O, (2) cis-aconitate + H2O = isocitrate. This reaction is the interconversion of citrate and isocitrate via the labile, enzyme-bound intermediate cis-aconitate. Water is removed from one part of the citrate molecule and added back to a different atom to form isocitrate.